{
  "gene_name": "Carboxypeptidase D",
  "term_id": "GO:0005615",
  "gene_symbol": "CPD",
  "gene": "UniProtKB:O75976",
  "term_label": "extracellular space"
}